negative regulation of cellular response to hypoxia [GO:1900038] (BP) Also known as: down regulation of cellular response to hypoxic stress, down regulation of cellular response to lowered oxygen tension, down-regulation of cellular response to hypoxic stress, down-regulation of cellular response to lowered oxygen tension, downregulation of cellular response to hypoxic stress, downregulation of cellular response to lowered oxygen tension, inhibition of cellular response to hypoxic stress, inhibition of cellular response to lowered oxygen tension, negative regulation of cellular response to hypoxic stress, negative regulation of cellular response to lowered oxygen tension, down regulation of cellular response to hypoxia, down-regulation of cellular response to hypoxia, downregulation of cellular response to hypoxia, inhibition of cellular response to hypoxia Subtypes: negative regulation of hypoxia-inducible factor-1alpha signaling pathway [GO:1902072], GO:1903298 Sources: GOC:TermGenie, GOC:yaf Relationships: is a type of negative regulation of cellular process [GO:0048523]; is a type of GO:0048585; is a type of regulation of cellular response to hypoxia [GO:1900037]; negatively regulates cellular response to hypoxia [GO:0071456] Definition: Any process that stops, prevents or reduces the frequency, rate or extent of cellular response to hypoxia.